{
  "term_id": "GO:0035567",
  "term_label": "non-canonical Wnt signaling pathway",
  "gene_symbol": "SFRP2",
  "gene": "UniProtKB:Q96HF1",
  "gene_name": "Secreted frizzled-related protein 2"
}